ubiquitin-dependent protein catabolic process via the multivesicular body sorting pathway [GO:0043162] (BP) References: PMID:11511343 Sources: GOC:jl Definition: The chemical reactions and pathways resulting in the breakdown of a protein or peptide covalently tagged with ubiquitin, via the multivesicular body (MVB) sorting pathway; ubiquitin-tagged proteins are sorted into MVBs, and delivered to a lysosome/vacuole for degradation. Relationships: is a type of ubiquitin-dependent protein catabolic process [GO:0006511]; has part protein catabolic process in the vacuole [GO:0007039]; has part GO:0071985 Also known as: ubiquitin-dependent protein breakdown via the multivesicular body pathway, ubiquitin-dependent protein catabolic process via the MVB pathway, ubiquitin-dependent protein catabolism via the MVB pathway, ubiquitin-dependent protein degradation via the multivesicular body pathway